{
  "gene": "UniProtKB:Q96I27",
  "term_id": "GO:0005634",
  "gene_symbol": "ZNF625",
  "gene_name": "Zinc finger protein 625",
  "term_label": "nucleus"
}